triglyceride storage [GO:0030730] (biological process) Also known as: retention of triacylglycerol, retention of triglyceride, sequestering of triacylglycerol, sequestering of triglyceride, sequestration of triacylglycerol, sequestration of triglyceride, storage of triacylglycerol, storage of triglyceride, triacylglycerol retention, triacylglycerol sequestering, triacylglycerol sequestration, triacylglycerol storage, triglyceride retention, triglyceride sequestering, triglyceride sequestration Definition: The process of binding or confining any triester of glycerol such that it is separated from other components of a biological system. Relationships: is a type of GO:0019915 Sources: GOC:mah, ISBN:0198506732 Regulation: regulated by regulation of triglyceride storage [GO:0010889]; positively regulated by GO:0010890; RO_0002212 by negative regulation of triglyceride storage [GO:0010891]